{
  "gene": "UniProtKB:Q9H2J4",
  "term_label": "protein folding",
  "gene_symbol": "PDCL3",
  "term_id": "GO:0006457",
  "gene_name": "Phosducin-like protein 3"
}